{
  "gene": "UniProtKB:Q8TDH9",
  "term_id": "UNKNOWN:0001",
  "term_label": "Unknown molecular function",
  "gene_name": "Biogenesis of lysosome-related organelles complex 1 subunit 5",
  "gene_symbol": "BLOC1S5"
}